dihydroorotase activity [GO:0004151] (MF) Definition: Catalysis of the reaction: (S)-dihydroorotate + H2O = N-carbamoyl-L-aspartate + H+. Also known as: (S)-dihydroorotate amidohydrolase activity, DHOase activity, carbamoylaspartic dehydrase activity, dihydroorotate hydrolase activity Relationships: is a type of hydrolase activity, acting on carbon-nitrogen (but not peptide) bonds, in cyclic amides [GO:0016812] Sources: EC:3.5.2.3, RHEA:24296